{
  "gene": "UniProtKB:Q7Z3V4",
  "gene_name": "Ubiquitin-protein ligase E3B",
  "term_id": "UNKNOWN:0003",
  "gene_symbol": "UBE3B",
  "term_label": "Unknown cellular component"
}